RNA polymerase I upstream activating factor complex [GO:0000500] (cellular component) Definition: A complex required for the transcription of rDNA by RNA polymerase I. In yeast the complex consists of Rrrn5p, Rrn9p, Rrn10p, histones H3 and H4, and Uaf30p. References: PMID:11500378 Also known as: RNA polymerase I upstream activation factor complex, UAF Relationships: is a type of RNA polymerase I transcription regulator complex [GO:0000120]